{
  "term_id": "GO:1902042",
  "gene": "UniProtKB:Q8WZ73",
  "gene_name": "E3 ubiquitin-protein ligase rififylin",
  "term_label": "negative regulation of extrinsic apoptotic signaling pathway via death domain receptors",
  "gene_symbol": "RFFL"
}